{
  "gene_name": "CUB and sushi domain-containing protein 1",
  "gene": "UniProtKB:Q96PZ7",
  "term_id": "UNKNOWN:0003",
  "term_label": "Unknown cellular component",
  "gene_symbol": "CSMD1"
}